{
  "gene_name": "Putative serine protease 46",
  "term_label": "Unknown molecular function",
  "gene_symbol": "PRSS46P",
  "gene": "UniProtKB:E5RG02",
  "term_id": "UNKNOWN:0001"
}